{
  "gene": "UniProtKB:Q6PJG9",
  "gene_name": "Leucine-rich repeat and fibronectin type-III domain-containing protein 4",
  "term_label": "cell surface",
  "term_id": "GO:0009986",
  "gene_symbol": "LRFN4"
}